extraglomerular mesangial cell proliferation [GO:0072122] (biological process) Also known as: Goormaghtigh proliferation, lacis cell proliferation Relationships: is_a GO:0072111; BFO_0000050 nephron development [GO:0072006] Subtypes: mesonephric extraglomerular mesangial cell proliferation involved in mesonephros development [GO:0061225], GO:0072261 Sources: GOC:mtg_kidney_jan10 Definition: The multiplication or reproduction of extraglomerular glomerular mesangium cells by cell division, resulting in the expansion of their population. Extraglomerular mesangial cells (also known as lacis cells, Goormaghtigh cells) are light-staining cells in the kidney found outside the glomerulus, near the vascular pole and macula densa.